regulation of L-tyrosine import across plasma membrane [GO:1900929] (biological process) Also known as: regulation of L-tyrosine import, regulation of L-tyrosine uptake Sources: GOC:TermGenie Definition: Any process that modulates the frequency, rate or extent of L-tyrosine import into the cell. Relationships: is a type of regulation of amino acid import across plasma membrane [GO:0010958]; is a type of regulation of organic acid transport [GO:0032890]; regulates L-tyrosine import across plasma membrane [GO:1903808] Subtypes: negative regulation of L-tyrosine import across plasma membrane [GO:1900930], positive regulation of L-tyrosine import across plasma membrane [GO:1900931]